endonucleolytic cleavage between SSU-rRNA and LSU-rRNA of tricistronic rRNA transcript (SSU-rRNA, LSU-rRNA, 5S) [GO:0000457] (biological process) Definition: Endonucleolytic cleavage to separate a pre-SSU-rRNA from a pre-LSU-rRNA originally produced as a tricistronic rRNA transcript that contains the Small Subunit (SSU) rRNA, the Large Subunit (LSU) rRNA, and the 5S rRNA, in that order, from 5' to 3' along the primary transcript. Note that the use of the word tricistronic refers only to the number of mature rRNA molecules which will be produced from the primary transcript and ignores tRNAs that may also be present within the primary transcript. Sources: GOC:curators Relationships: is a type of GO:0000449; is part of maturation of LSU-rRNA from tricistronic rRNA transcript (SSU-rRNA, LSU-rRNA,5S) [GO:0002108]; is part of maturation of SSU-rRNA from tricistronic rRNA transcript (SSU-rRNA, LSU-rRNA,5S) [GO:0002109]